phosphorelay sensor kinase activity [GO:0000155] (molecular function) References: PMID:10966457, PMID:20223701, PMID:31386843, PMID:9191038 Sources: GOC:bf, GOC:mcc Also known as: two-component sensor activity, two-component sensor molecule, two-component system sensor activity Definition: Catalysis of the phosphorylation of a histidine residue in response to detection of an extracellular signal such as a chemical ligand or change in environment, to initiate a change in cell state or activity. The two-component sensor is a histidine kinase that autophosphorylates a histidine residue in its active site. The phosphate is then transferred to an aspartate residue in a downstream response regulator, to trigger a response. Relationships: is_a protein histidine kinase activity [GO:0004673]; is a type of molecular sensor activity [GO:0140299]; BFO_0000050 phosphorelay signal transduction system [GO:0000160]